{
  "gene_name": "FAST kinase domain-containing protein 4",
  "gene": "UniProtKB:Q969Z0",
  "term_label": "mitochondrial RNA processing",
  "term_id": "GO:0000963",
  "gene_symbol": "TBRG4"
}